{
  "term_id": "UNKNOWN:0002",
  "gene": "UniProtKB:Q9C0I9",
  "term_label": "Unknown biological process",
  "gene_name": "Leucine-rich repeat-containing protein 27",
  "gene_symbol": "LRRC27"
}